megakaryocyte differentiation [GO:0030219] (biological process) Also known as: megakaryocyte cell differentiation Definition: The process in which a myeloid precursor cell acquires specializes features of a megakaryocyte. Regulation: regulated by regulation of megakaryocyte differentiation [GO:0045652]; negatively regulated by negative regulation of megakaryocyte differentiation [GO:0045653]; positively regulated by GO:0045654 Relationships: is a type of myeloid cell differentiation [GO:0030099] Sources: GOC:mah